{
  "gene_name": "Suppressor of cytokine signaling 6",
  "gene_symbol": "SOCS6",
  "term_label": "Unknown biological process",
  "gene": "UniProtKB:O14544",
  "term_id": "UNKNOWN:0002"
}